{
  "gene_symbol": "TBC1D9",
  "gene_name": "TBC1 domain family member 9",
  "term_label": "Unknown biological process",
  "term_id": "UNKNOWN:0002",
  "gene": "UniProtKB:Q6ZT07"
}